{
  "term_id": "GO:0003730",
  "gene": "UniProtKB:Q9NR90",
  "term_label": "mRNA 3'-UTR binding",
  "gene_symbol": "DAZ3",
  "gene_name": "Deleted in azoospermia protein 3"
}